negative regulation of protein localization to chromatin [GO:0120186] (biological process) Also known as: negative regulation of protein localisation to chromatin Definition: Any process that stops, prevents, or reduces the frequency, rate or extent of protein localization to chromatin. Relationships: is a type of negative regulation of protein localization [GO:1903828]; is_a GO:1905634; negatively regulates protein localization to chromatin [GO:0071168] References: PMID:20889714, PMID:29899453